{
  "term_id": "GO:0016477",
  "term_label": "cell migration",
  "gene_symbol": "FSCN1",
  "gene_name": "Fascin",
  "gene": "UniProtKB:Q16658"
}